{
  "gene_symbol": "BACE1",
  "term_label": "trans-Golgi network",
  "gene_name": "Beta-secretase 1",
  "gene": "UniProtKB:P56817",
  "term_id": "GO:0005802"
}